{
  "term_label": "Unknown molecular function",
  "gene_symbol": "ZMYND11",
  "gene_name": "Zinc finger MYND domain-containing protein 11",
  "gene": "UniProtKB:Q15326",
  "term_id": "UNKNOWN:0001"
}